umbilical cord development [GO:0061027] (BP) Sources: GOC:BHF, GOC:dph Definition: The process whose specific outcome is the development of the umbilical cord, from its formation to the mature structure. The umbilical cord is an organ or embryonic origin consisting of the 2 umbilical arteries and the one umbilical vein. The umbilical cord connects the cardiovascular system of the fetus to the mother via the placenta. Relationships: is a type of anatomical structure development [GO:0048856]